lateral line ganglion neuron differentiation [GO:0048891] (biological process) References: PMID:15018940 Subtypes: anterior lateral line ganglion neuron differentiation [GO:0048908], posterior lateral line ganglion neuron differentiation [GO:0048928] Also known as: gLL neuron differentiation Definition: The process in which a relatively unspecialized cell acquires specialized features of a lateral line ganglion neuron. Relationships: is a type of peripheral nervous system neuron differentiation [GO:0048934]; BFO_0000050 lateral line ganglion development [GO:0048890]